pexophagosome [GO:1990457] (cellular component) Relationships: is a type of phagocytic vesicle [GO:0045335] Definition: A membrane-bounded intracellular vesicle involved in the degradation of peroxisome by macropexophagy. References: PMID:22536249